{
  "term_id": "GO:0016323",
  "term_label": "basolateral plasma membrane",
  "gene": "UniProtKB:P78310",
  "gene_symbol": "CXADR",
  "gene_name": "Coxsackievirus and adenovirus receptor"
}